{
  "term_label": "chromosome segregation",
  "term_id": "GO:0007059",
  "gene_name": "Nuclear distribution protein nudE-like 1",
  "gene": "UniProtKB:Q9GZM8",
  "gene_symbol": "NDEL1"
}